{
  "gene_symbol": "RASSF5",
  "term_label": "signal transduction",
  "gene": "UniProtKB:Q8WWW0",
  "gene_name": "Ras association domain-containing protein 5",
  "term_id": "GO:0007165"
}